{
  "term_label": "cytosol",
  "gene_name": "Inositol hexakisphosphate and diphosphoinositol-pentakisphosphate kinase 2",
  "gene_symbol": "PPIP5K2",
  "gene": "UniProtKB:O43314",
  "term_id": "GO:0005829"
}